{
  "term_id": "GO:0005432",
  "gene": "UniProtKB:P57103",
  "gene_symbol": "SLC8A3",
  "gene_name": "Sodium_calcium exchanger 3",
  "term_label": "calcium:sodium antiporter activity"
}